{
  "gene": "UniProtKB:Q9UBF8",
  "term_label": "membrane",
  "gene_symbol": "PI4KB",
  "term_id": "GO:0016020",
  "gene_name": "Phosphatidylinositol 4-kinase beta"
}